{
  "gene": "UniProtKB:E0CX11",
  "gene_name": "Short transmembrane mitochondrial protein 1",
  "gene_symbol": "STMP1",
  "term_id": "GO:0098803",
  "term_label": "respiratory chain complex"
}